RNA-protein covalent cross-linking via peptidyl-serine [GO:0018259] (biological process) Relationships: is a type of RNA-protein covalent cross-linking [GO:0018144]; is a type of peptidyl-serine modification [GO:0018209] Sources: RESID:AA0213 Definition: The formation of a covalent cross-link between RNA and a peptidyl-serine residue by the formation of O-(phospho-5'-5NA)-L-serine.